regulation of response to cycloalkane [GO:1901431] (biological process) Sources: GOC:TermGenie, GOC:mengo_curators Subtypes: negative regulation of response to cycloalkane [GO:1901432], positive regulation of response to cycloalkane [GO:1901433] Relationships: is a type of GO:0048583; regulates response to cycloalkane [GO:0014071] Definition: Any process that modulates the frequency, rate or extent of response to cycloalkane.